determination of wing disc primordium [GO:0035294] (biological process) Relationships: is a type of determination of imaginal disc primordium [GO:0007445]; is a type of wing disc development [GO:0035220] Definition: Allocation of embryonic cells to the wing disc founder populations, groups of cells that are committed to contribute to the formation of a wing imaginal disc. Sources: ISBN:0879694238